{
  "term_id": "UNKNOWN:0001",
  "term_label": "Unknown molecular function",
  "gene_name": "Olfactory receptor 8J3",
  "gene_symbol": "OR8J3",
  "gene": "UniProtKB:Q8NGG0"
}